{
  "gene_symbol": "SLCO1A2",
  "gene": "UniProtKB:P46721",
  "term_id": "GO:0016323",
  "gene_name": "Solute carrier organic anion transporter family member 1A2",
  "term_label": "basolateral plasma membrane"
}